{
  "gene_symbol": "H1-0",
  "gene": "UniProtKB:P07305",
  "term_label": "double-stranded DNA binding",
  "term_id": "GO:0003690",
  "gene_name": "Histone H1.0"
}